{
  "term_label": "Unknown cellular component",
  "gene": "UniProtKB:Q8N268",
  "gene_symbol": "LINC02910",
  "term_id": "UNKNOWN:0003",
  "gene_name": "Putative uncharacterized protein encoded by LINC02910"
}